amino acid catabolic process to alcohol via Ehrlich pathway [GO:0000947] (biological process) Definition: The chemical reactions and pathways involving the catabolism of amino acids to produce alcohols with one carbon less than the starting amino acid. In S. cerevisiae, this is known to occur for leucine, isoleucine, valine, methionine, phenylalanine, tyrosine, or tryptophan. Often referred to as the Ehrlich pathway, these reactions generally occur during fermentation to produce a variety of alcohols, often collectively referred to as fusel alcohols. Depending on the redox state of the cells, carboxylic acid derivatives may be produced instead of alcohols. References: PMID:18281432 Sources: GOC:krc Relationships: is_a GO:0000955; is a type of GO:0046165 Subtypes: aromatic amino acid family catabolic process to alcohol via Ehrlich pathway [GO:0000949], GO:0000950, L-methionine catabolic process to 3-methylthiopropanol [GO:0000951]